{
  "gene_name": "Centromere protein R",
  "term_label": "Unknown molecular function",
  "gene_symbol": "ITGB3BP",
  "gene": "UniProtKB:Q13352",
  "term_id": "UNKNOWN:0001"
}